{
  "term_label": "regulation of transcription by RNA polymerase II",
  "gene": "UniProtKB:Q9H175",
  "gene_name": "Cysteine_serine-rich nuclear protein 2",
  "term_id": "GO:0006357",
  "gene_symbol": "CSRNP2"
}